{
  "term_id": "GO:0007271",
  "gene_name": "Neuronal acetylcholine receptor subunit alpha-3",
  "term_label": "synaptic transmission, cholinergic",
  "gene_symbol": "CHRNA3",
  "gene": "UniProtKB:P32297"
}